oxidoreductase activity, acting on paired donors, with incorporation or reduction of molecular oxygen, reduced pteridine as one donor, and incorporation of one atom of oxygen [GO:0016714] (molecular function) Subtypes: phenylalanine 4-monooxygenase activity [GO:0004505], GO:0004510, tyrosine 3-monooxygenase activity [GO:0004511], GO:0050479, mandelate 4-monooxygenase activity [GO:0050481] Relationships: is a type of monooxygenase activity [GO:0004497]; is a type of oxidoreductase activity, acting on paired donors, with incorporation or reduction of molecular oxygen [GO:0016705] Sources: EC:1.14.16.- Definition: Catalysis of an oxidation-reduction (redox) reaction in which hydrogen or electrons are transferred from reduced pteridine and one other donor, and one atom of oxygen is incorporated into one donor.